{
  "gene_symbol": "IL11",
  "term_id": "GO:0005125",
  "gene": "UniProtKB:P20809",
  "term_label": "cytokine activity",
  "gene_name": "Interleukin-11"
}